{
  "term_label": "Unknown biological process",
  "gene_name": "Protein maestro",
  "gene": "UniProtKB:Q9BYG7",
  "term_id": "UNKNOWN:0002",
  "gene_symbol": "MRO"
}